pons development [GO:0021548] (biological process) Definition: The process whose specific outcome is the progression of the pons over time, from its formation to the mature structure. The pons lies above the medulla and next to the cerebellum. The pons conveys information about movement from the cerebral hemisphere to the cerebellum. Relationships: is a type of anatomical structure development [GO:0048856]; is part of metencephalon development [GO:0022037] Sources: GOC:cls, GOC:dgh, GOC:dph, GOC:jid, GO_REF:0000021